{
  "term_label": "nucleus",
  "gene": "UniProtKB:Q5H9F3",
  "gene_name": "BCL-6 corepressor-like protein 1",
  "gene_symbol": "BCORL1",
  "term_id": "GO:0005634"
}